proteasome regulatory particle binding [GO:1904855] (molecular function) Also known as: PA700-dependent proteasome activator binding, 19S regulatory particle binding, PA700 proteasome activator binding, modulator complex binding References: PMID:16096059 Sources: GOC:TermGenie Definition: Binding to a proteasome regulatory particle. Relationships: is a type of protein-containing complex binding [GO:0044877]